{
  "gene_name": "Mitogen-activated protein kinase kinase kinase 7",
  "term_label": "positive regulation of canonical NF-kappaB signal transduction",
  "gene_symbol": "MAP3K7",
  "term_id": "GO:0043123",
  "gene": "UniProtKB:O43318"
}